{
  "gene": "UniProtKB:Q1A5X7",
  "term_label": "Unknown cellular component",
  "gene_name": "Putative WASP homolog-associated protein with actin, membranes and microtubules-like protein 1",
  "term_id": "UNKNOWN:0003",
  "gene_symbol": "WHAMMP3"
}